venous endothelial cell fate commitment [GO:0060845] (biological process) Definition: The commitment of a cell to a venous endothelial cell fate and its capacity to differentiate into an venous endothelial cell. Relationships: is a type of GO:0060846; is part of venous endothelial cell differentiation [GO:0060843] Sources: GOC:dph, GOC:sdb_2009, GOC:tb Regulation: regulated by GO:2000787; negatively regulated by negative regulation of venous endothelial cell fate commitment [GO:2000788]; positively regulated by positive regulation of venous endothelial cell fate commitment [GO:2000789]